{
  "term_id": "GO:0050911",
  "gene_symbol": "OR2W3",
  "gene_name": "Olfactory receptor 2W3",
  "term_label": "detection of chemical stimulus involved in sensory perception of smell",
  "gene": "UniProtKB:Q7Z3T1"
}